lipid droplet disassembly [GO:1905691] (biological process) Also known as: adiposome disassembly, lipid body disassembly, lipid droplet reserve breakdown, lipid particle disassembly Definition: The disaggregation of a lipid particle into its constituent components. Relationships: is a type of lipid droplet organization [GO:0034389]; is a type of GO:1903008 Sources: GOC:TermGenie, GOC:autophagy, GOC:pr, GO_REF:0000079